{
  "gene_symbol": "FRMD1",
  "gene": "UniProtKB:Q8N878",
  "gene_name": "FERM domain-containing protein 1",
  "term_label": "protein sequestering activity",
  "term_id": "GO:0140311"
}